{
  "gene_symbol": "CYB5R2",
  "gene_name": "NADH-cytochrome b5 reductase 2",
  "gene": "UniProtKB:Q6BCY4",
  "term_id": "GO:0071949",
  "term_label": "FAD binding"
}